{
  "gene": "UniProtKB:Q15274",
  "term_id": "GO:0009435",
  "gene_symbol": "QPRT",
  "term_label": "NAD+ biosynthetic process",
  "gene_name": "Nicotinate-nucleotide pyrophosphorylase [carboxylating]"
}